acetylene hydratase activity [GO:0018818] (molecular function) Definition: Catalysis of the reaction: acetaldehyde = acetylene + H2O. Sources: EC:4.2.1.112, RHEA:17885 Also known as: AH, AHy, acetaldehyde hydro-lyase activity Relationships: is a type of hydro-lyase activity [GO:0016836]